{
  "gene_symbol": "TMCC1",
  "gene_name": "Transmembrane and coiled-coil domains protein 1",
  "gene": "UniProtKB:O94876",
  "term_id": "GO:0090148",
  "term_label": "membrane fission"
}